tubuloglomerular feedback [GO:0003098] (biological process) Definition: The process in which blood volume is regulated due to a change in the rate of glomerular filtration. This is accomplished by a feedback mechanism that senses changes in the juxtaglomerular apparatus. Sources: GOC:mtg_cardio Relationships: is a type of renal system process involved in regulation of blood volume [GO:0001977]; is part of GO:0003093